dimethyl sulfoxide reductase activity [GO:0009389] (molecular function) Definition: Catalysis of the reaction: dimethyl sulfoxide + H+ = dimethyl sulfide + H2O. Also known as: dimethyl sulphoxide reductase activity References: PMID:8658134 Relationships: is_a oxidoreductase activity, acting on a sulfur group of donors [GO:0016667]